negative regulation of paraxial mesodermal cell fate determination [GO:0048347] (biological process) Also known as: down regulation of paraxial mesodermal cell fate determination, down-regulation of paraxial mesodermal cell fate determination, downregulation of paraxial mesodermal cell fate determination, inhibition of paraxial mesodermal cell fate determination Definition: Any process that stops, prevents, or reduces the frequency, rate or extent of paraxial mesoderm cell fate determination. Sources: GOC:dgh Relationships: is a type of negative regulation of mesodermal cell fate determination [GO:0048335]; is a type of GO:0048345; negatively regulates paraxial mesodermal cell fate determination [GO:0048344]